{
  "term_label": "nucleus",
  "term_id": "GO:0005634",
  "gene": "UniProtKB:Q6FI13",
  "gene_name": "Histone H2A type 2-A",
  "gene_symbol": "H2AC19"
}